{
  "gene_name": "Interferon-induced protein 44-like",
  "term_id": "GO:0006955",
  "gene_symbol": "IFI44L",
  "term_label": "immune response",
  "gene": "UniProtKB:Q53G44"
}